{
  "term_label": "Unknown cellular component",
  "gene": "UniProtKB:Q03154",
  "gene_symbol": "ACY1",
  "term_id": "UNKNOWN:0003",
  "gene_name": "Aminoacylase-1"
}